{
  "gene": "UniProtKB:Q8IWK6",
  "gene_name": "Adhesion G protein-coupled receptor A3",
  "term_label": "cell surface receptor signaling pathway",
  "term_id": "GO:0007166",
  "gene_symbol": "ADGRA3"
}